{
  "gene_symbol": "MFSD8",
  "term_label": "lysosome organization",
  "term_id": "GO:0007040",
  "gene": "UniProtKB:Q8NHS3",
  "gene_name": "Major facilitator superfamily domain-containing protein 8"
}